{
  "gene_symbol": "IL10RB",
  "gene": "UniProtKB:Q08334",
  "gene_name": "Interleukin-10 receptor subunit beta",
  "term_id": "GO:0019221",
  "term_label": "cytokine-mediated signaling pathway"
}